{
  "gene_symbol": "ME2",
  "term_id": "GO:0005739",
  "term_label": "mitochondrion",
  "gene_name": "NAD-dependent malic enzyme, mitochondrial",
  "gene": "UniProtKB:P23368"
}